apicoplast [GO:0020011] (cellular component) Relationships: is a type of plastid [GO:0009536] Definition: The plastid organelle found in apicomplexans. Sources: ISBN:0521664470